{
  "gene_symbol": "UCK2",
  "term_id": "GO:0005737",
  "gene": "UniProtKB:Q9BZX2",
  "term_label": "cytoplasm",
  "gene_name": "Uridine-cytidine kinase 2"
}